{
  "term_label": "Unknown molecular function",
  "gene_symbol": "A0A8I5QKQ9",
  "gene_name": "Uncharacterized protein",
  "gene": "UniProtKB:A0A8I5QKQ9",
  "term_id": "UNKNOWN:0001"
}